{
  "gene": "UniProtKB:Q5JST6",
  "gene_symbol": "EFHC2",
  "gene_name": "EF-hand domain-containing family member C2",
  "term_label": "Unknown molecular function",
  "term_id": "UNKNOWN:0001"
}